{
  "term_label": "negative regulation of metaphase/anaphase transition of meiotic cell cycle",
  "gene_name": "Proto-oncogene serine_threonine-protein kinase mos",
  "gene_symbol": "MOS",
  "gene": "UniProtKB:P00540",
  "term_id": "GO:1902103"
}